{
  "term_id": "GO:0005829",
  "term_label": "cytosol",
  "gene_name": "Rab5 GDP_GTP exchange factor",
  "gene": "UniProtKB:Q9UJ41",
  "gene_symbol": "RABGEF1"
}